sialic acid transport [GO:0015739] (biological process) Relationships: is a type of carboxylic acid transport [GO:0046942] Sources: GOC:krc Definition: The directed movement of sialic acid into, out of or within a cell, or between cells, by means of some agent such as a transporter or pore.